{
  "gene": "UniProtKB:Q7Z340",
  "term_label": "DNA-binding transcription factor activity, RNA polymerase II-specific",
  "term_id": "GO:0000981",
  "gene_name": "Zinc finger protein 551",
  "gene_symbol": "ZNF551"
}